{
  "term_label": "Unknown cellular component",
  "gene": "UniProtKB:Q8NHY0",
  "gene_symbol": "B4GALNT2",
  "gene_name": "Beta-1,4 N-acetylgalactosaminyltransferase 2",
  "term_id": "UNKNOWN:0003"
}